{
  "gene_symbol": "KCNG4",
  "gene_name": "Potassium voltage-gated channel subfamily G member 4",
  "gene": "UniProtKB:Q8TDN1",
  "term_id": "GO:0071805",
  "term_label": "potassium ion transmembrane transport"
}